{
  "gene_name": "DNA mismatch repair protein Mlh1",
  "gene": "UniProtKB:P40692",
  "gene_symbol": "MLH1",
  "term_id": "GO:0006298",
  "term_label": "mismatch repair"
}